{
  "gene": "UniProtKB:Q9NQN1",
  "term_id": "GO:0050911",
  "term_label": "detection of chemical stimulus involved in sensory perception of smell",
  "gene_name": "Olfactory receptor 2S2",
  "gene_symbol": "OR2S2"
}